xylem-to-phloem iron transport [GO:1990388] (BP) Relationships: is a type of iron ion transport [GO:0006826]; is a type of phloem transport [GO:0010233] References: PMID:24867923 Sources: GOC:tb Definition: The directed movement of iron ions into the phloem from the xylem.